{
  "gene": "UniProtKB:Q15125",
  "term_label": "C-8 sterol isomerase activity",
  "gene_name": "3-beta-hydroxysteroid-Delta(8),Delta(7)-isomerase",
  "gene_symbol": "EBP",
  "term_id": "GO:0000247"
}